fibronectin binding [GO:0001968] (molecular function) Definition: Binding to a fibronectin, a group of related adhesive glycoproteins of high molecular weight found on the surface of animal cells, connective tissue matrices, and in extracellular fluids. Sources: GOC:hjd Relationships: is a type of protein binding [GO:0005515]